{
  "term_id": "GO:0006289",
  "gene": "UniProtKB:P78549",
  "gene_name": "Endonuclease III-like protein 1",
  "gene_symbol": "NTHL1",
  "term_label": "nucleotide-excision repair"
}